{
  "term_id": "GO:0000981",
  "gene_symbol": "MIXL1",
  "gene": "UniProtKB:Q9H2W2",
  "gene_name": "Homeobox protein MIXL1",
  "term_label": "DNA-binding transcription factor activity, RNA polymerase II-specific"
}